regulation of synaptic transmission, cholinergic [GO:0032222] (biological process) Definition: Any process that modulates the frequency, rate or extent of cholinergic synaptic transmission, the process of communication from a neuron to another neuron across a synapse using the neurotransmitter acetylcholine. Sources: GOC:mah Subtypes: regulation of acetylcholine secretion, neurotransmission [GO:0014056], negative regulation of synaptic transmission, cholinergic [GO:0032223], positive regulation of synaptic transmission, cholinergic [GO:0032224] Relationships: is a type of modulation of chemical synaptic transmission [GO:0050804]; regulates synaptic transmission, cholinergic [GO:0007271]